{
  "gene_name": "Epsin-3",
  "term_id": "GO:0005886",
  "gene": "UniProtKB:Q9H201",
  "term_label": "plasma membrane",
  "gene_symbol": "EPN3"
}